tRNA-specific adenosine-34 deaminase activity [GO:0052717] (molecular function) References: PMID:17875641 Sources: RHEA:43168 Definition: Catalysis of the reaction: adenosine-34 + H2O = inosine-34 + NH3, in a tRNA-Ala molecule. Also known as: tRNA(Ala)-A34 deaminase activity Relationships: is a type of GO:0008251